lipid-linked peptidoglycan transporter activity [GO:0015648] (MF) Definition: Enables the directed movement of lipid-linked peptidoglycans into, out of or within a cell, or between cells. Also known as: lipid-linked murein transporter activity Relationships: is a type of GO:0015647; is part of lipid-linked peptidoglycan transport [GO:0015836] Sources: GOC:mah